{
  "gene": "UniProtKB:Q8N5C8",
  "term_label": "positive regulation of canonical NF-kappaB signal transduction",
  "term_id": "GO:0043123",
  "gene_name": "TGF-beta-activated kinase 1 and MAP3K7-binding protein 3",
  "gene_symbol": "TAB3"
}